{
  "gene": "UniProtKB:O75955",
  "term_label": "positive regulation of endocytosis",
  "term_id": "GO:0045807",
  "gene_name": "Flotillin-1",
  "gene_symbol": "FLOT1"
}